{
  "term_id": "UNKNOWN:0001",
  "gene_name": "Transmembrane and coiled-coil domain-containing protein 6",
  "term_label": "Unknown molecular function",
  "gene_symbol": "TMCO6",
  "gene": "UniProtKB:Q96DC7"
}